{
  "gene_name": "Arf-GAP with coiled-coil, ANK repeat and PH domain-containing protein 3",
  "term_label": "Unknown biological process",
  "gene_symbol": "ACAP3",
  "gene": "UniProtKB:Q96P50",
  "term_id": "UNKNOWN:0002"
}